{
  "gene": "UniProtKB:Q5T6C5",
  "gene_name": "Ataxin-7-like protein 2",
  "term_label": "Unknown molecular function",
  "term_id": "UNKNOWN:0001",
  "gene_symbol": "ATXN7L2"
}